{
  "gene_symbol": "PRR23D2",
  "gene": "UniProtKB:P0DMB1",
  "term_id": "UNKNOWN:0003",
  "term_label": "Unknown cellular component",
  "gene_name": "Proline-rich protein 23D2"
}